bioluminescence [GO:0008218] (biological process) Sources: ISBN:0198506732 Definition: The production of light by certain enzyme-catalyzed reactions in cells. Relationships: is a type of metabolic process [GO:0008152] Regulation: RO_0002211 by regulation of bioluminescence [GO:1905085]; negatively regulated by negative regulation of bioluminescence [GO:1905086]; positively regulated by positive regulation of bioluminescence [GO:1905087]